{
  "term_id": "GO:0007167",
  "gene_name": "CNK3_IPCEF1 fusion protein",
  "gene_symbol": "CNK3/IPCEF1",
  "gene": "UniProtKB:G9CGD6",
  "term_label": "enzyme-linked receptor protein signaling pathway"
}